{
  "term_id": "GO:0005615",
  "gene_name": "Serine protease 33",
  "gene": "UniProtKB:Q8NF86",
  "term_label": "extracellular space",
  "gene_symbol": "PRSS33"
}